{
  "gene_name": "E3 ubiquitin-protein ligase E3D",
  "gene_symbol": "UBE3D",
  "gene": "UniProtKB:Q7Z6J8",
  "term_label": "proteasome-mediated ubiquitin-dependent protein catabolic process",
  "term_id": "GO:0043161"
}